positive regulation of RNA biosynthetic process [GO:1902680] (biological process) Also known as: positive regulation of RNA anabolism, positive regulation of RNA biosynthesis, positive regulation of RNA formation, positive regulation of RNA synthesis, up regulation of RNA anabolism, up regulation of RNA biosynthesis, up regulation of RNA biosynthetic process, up regulation of RNA formation, up regulation of RNA synthesis, up-regulation of RNA anabolism, up-regulation of RNA biosynthesis, up-regulation of RNA biosynthetic process, up-regulation of RNA formation, up-regulation of RNA synthesis, upregulation of RNA anabolism, upregulation of RNA biosynthesis, upregulation of RNA biosynthetic process, upregulation of RNA formation, upregulation of RNA synthesis, activation of RNA anabolism, activation of RNA biosynthesis, activation of RNA biosynthetic process, activation of RNA formation, activation of RNA synthesis Definition: Any process that activates or increases the frequency, rate or extent of RNA biosynthetic process. Subtypes: positive regulation of single stranded viral RNA replication via double stranded DNA intermediate [GO:0045870], positive regulation of DNA-templated transcription [GO:0045893], positive regulation of promoter clearance from RNA polymerase II promoter [GO:0140846] Sources: GO:jl, GOC:TermGenie, GO_REF:0000058 Relationships: is a type of positive regulation of macromolecule biosynthetic process [GO:0010557]; is a type of positive regulation of RNA metabolic process [GO:0051254]; is a type of regulation of RNA biosynthetic process [GO:2001141]; positively regulates RNA biosynthetic process [GO:0032774]